{
  "gene_symbol": "PTPRCAP",
  "term_label": "plasma membrane",
  "term_id": "GO:0005886",
  "gene_name": "Protein tyrosine phosphatase receptor type C-associated protein",
  "gene": "UniProtKB:Q14761"
}